{
  "term_label": "synaptic vesicle fusion to presynaptic active zone membrane",
  "gene_name": "Proline-rich transmembrane protein 2",
  "gene_symbol": "PRRT2",
  "term_id": "GO:0031629",
  "gene": "UniProtKB:Q7Z6L0"
}